{
  "gene_symbol": "SURF2",
  "term_id": "UNKNOWN:0003",
  "gene_name": "Surfeit locus protein 2",
  "term_label": "Unknown cellular component",
  "gene": "UniProtKB:Q15527"
}